dopamine secretion, neurotransmission [GO:0061527] (biological process) Definition: The regulated release of dopamine by a cell in which the dopamine acts as a neurotransmitter. Sources: GOC:dph Relationships: is a type of axonal dopamine secretion [GO:0099124]; is a type of catecholamine secretion, neurotransmission [GO:0160043]; is part of GO:0001963